{
  "gene": "UniProtKB:Q8IWN6",
  "term_id": "UNKNOWN:0001",
  "gene_name": "Protein FAM223A",
  "gene_symbol": "FAM223A",
  "term_label": "Unknown molecular function"
}